regulation of serotonin secretion [GO:0014062] (biological process) Also known as: regulation of serotonin release Subtypes: negative regulation of serotonin secretion [GO:0014063], positive regulation of serotonin secretion [GO:0014064] Sources: GOC:ef Definition: Any process that modulates the frequency, rate or extent of the regulated release of serotonin. Relationships: is_a GO:0043269; is a type of regulation of secretion by cell [GO:1903530]; RO_0002211 GO:0001820